{
  "term_label": "Unknown molecular function",
  "gene": "UniProtKB:Q9NX14",
  "gene_name": "NADH dehydrogenase [ubiquinone] 1 beta subcomplex subunit 11, mitochondrial",
  "gene_symbol": "NDUFB11",
  "term_id": "UNKNOWN:0001"
}